{
  "gene_symbol": "JAK2",
  "gene": "UniProtKB:O60674",
  "term_label": "cytokine-mediated signaling pathway",
  "term_id": "GO:0019221",
  "gene_name": "Tyrosine-protein kinase JAK2"
}